nodal receptor complex assembly [GO:0038099] (biological process) Relationships: is a type of protein-containing complex assembly [GO:0065003]; is part of nodal signaling pathway [GO:0038092] Regulation: regulated by regulation of nodal receptor complex assembly [GO:1900123]; negatively regulated by negative regulation of nodal receptor complex assembly [GO:1900124] References: PMID:15062104 Sources: GOC:bf, GOC:signaling Definition: The aggregation, arrangement and bonding together of a set of components to form a complex containing a type II activin receptor, a type I activin receptor, and a coreceptor of the EGF-CFC family (e.g. Cripto or Cryptic, in mammals). Also known as: ActRIIB.ALK4.EGF-CFC complex formation, nodal receptor complex formation